{
  "gene": "UniProtKB:P0C7N8",
  "gene_symbol": "OR9G9",
  "gene_name": "Olfactory receptor 9G9",
  "term_label": "Unknown cellular component",
  "term_id": "UNKNOWN:0003"
}